{
  "term_label": "Unknown cellular component",
  "term_id": "UNKNOWN:0003",
  "gene": "UniProtKB:Q9NQG5",
  "gene_name": "Regulation of nuclear pre-mRNA domain-containing protein 1B",
  "gene_symbol": "RPRD1B"
}